butyryl-CoA biosynthetic process [GO:0044578] (biological process) Sources: GOC:jl Also known as: butyryl-CoA biosynthesis Relationships: is a type of fatty acid biosynthetic process [GO:0006633]; is a type of fatty-acyl-CoA biosynthetic process [GO:0046949] Subtypes: butyryl-CoA biosynthetic process from acetyl-CoA [GO:0044579] Definition: The chemical reactions and pathway resulting in the formation of butyryl-CoA.